{
  "gene_symbol": "AKAP5",
  "term_id": "GO:0031698",
  "term_label": "beta-2 adrenergic receptor binding",
  "gene": "UniProtKB:P24588",
  "gene_name": "A-kinase anchor protein 5"
}